fluoroacetaldehyde dehydrogenase (NAD+) activity [GO:0033723] (molecular function) Also known as: fluoroacetaldehyde:NAD+ oxidoreductase activity Relationships: is a type of GO:0004029 Sources: EC:1.2.1.69 Definition: Catalysis of the reaction: fluoroacetaldehyde + NAD+ + H2O = fluoroacetate + NADH + 2 H+.